{
  "gene_symbol": "C1orf87",
  "gene_name": "Uncharacterized protein C1orf87",
  "term_label": "Unknown molecular function",
  "gene": "UniProtKB:Q8N0U7",
  "term_id": "UNKNOWN:0001"
}